leucyl-tRNA aminoacylation [GO:0006429] (biological process) Definition: The process of coupling leucine to leucyl-tRNA, catalyzed by leucyl-tRNA synthetase. The leucyl-tRNA synthetase is a class-I synthetase. The activated amino acid is transferred to the 2'-OH group of a leucine-accetping tRNA. The 2'-O-aminoacyl-tRNA will ultimately migrate to the 3' position via transesterification. Subtypes: mitochondrial leucyl-tRNA aminoacylation [GO:0070153] Relationships: is a type of tRNA aminoacylation for protein translation [GO:0006418] Sources: GOC:mcc, ISBN:0716730510